positive regulation of cellulose biosynthetic process [GO:2001008] (biological process) Subtypes: positive regulation of plant-type cell wall cellulose biosynthetic process [GO:2001011] Sources: GOC:mengo_curators Also known as: positive regulation of cellulose anabolism, positive regulation of cellulose biosynthesis, positive regulation of cellulose formation, positive regulation of cellulose synthesis Relationships: is a type of positive regulation of macromolecule biosynthetic process [GO:0010557]; is_a GO:0045913; is a type of regulation of cellulose biosynthetic process [GO:2001006]; positively regulates cellulose biosynthetic process [GO:0030244] Definition: Any process that activates or increases the frequency, rate or extent of cellulose biosynthetic process.